apical distal dendrite [GO:0150014] (cellular component) Relationships: is a type of GO:0097440; is a type of distal dendrite [GO:0150002] References: PMID:1720142, PMID:20629984, PMID:9214543 Sources: GO:bc, GOC:aruk Definition: Any dendrite in a dendritic tree that emerges near the apical pole of a neuron, and which is farthest away from the neuronal cell body (the soma).